{
  "term_id": "GO:0034316",
  "gene_name": "Glia maturation factor gamma",
  "term_label": "negative regulation of Arp2/3 complex-mediated actin nucleation",
  "gene_symbol": "GMFG",
  "gene": "UniProtKB:O60234"
}